{
  "gene": "UniProtKB:O95264",
  "gene_name": "5-hydroxytryptamine receptor 3B",
  "term_id": "GO:1904315",
  "gene_symbol": "HTR3B",
  "term_label": "transmitter-gated monoatomic ion channel activity involved in regulation of postsynaptic membrane potential"
}